{
  "gene_name": "LASP1 neighbor protein",
  "term_id": "UNKNOWN:0003",
  "gene_symbol": "LASP1NB",
  "gene": "UniProtKB:A0A1B0GWH6",
  "term_label": "Unknown cellular component"
}